{
  "gene_name": "General transcription factor II-I repeat domain-containing protein 2A",
  "term_id": "GO:0005634",
  "gene_symbol": "GTF2IRD2",
  "gene": "UniProtKB:Q86UP8",
  "term_label": "nucleus"
}